{
  "gene_symbol": "SUGCT",
  "term_label": "succinate-hydroxymethylglutarate CoA-transferase activity",
  "gene": "UniProtKB:Q9HAC7",
  "term_id": "GO:0047369",
  "gene_name": "Succinate--hydroxymethylglutarate CoA-transferase"
}